regulation of glutamine transport [GO:2000485] (biological process) Also known as: regulation of L-glutamine transport Sources: GOC:obol Subtypes: regulation of L-glutamine import across plasma membrane [GO:1901034], negative regulation of glutamine transport [GO:2000486], GO:2000487 Relationships: is a type of GO:0032890; is a type of regulation of amino acid transport [GO:0051955]; regulates glutamine transport [GO:0006868] Definition: Any process that modulates the frequency, rate or extent of glutamine transport.